{
  "term_id": "GO:0008083",
  "gene_name": "Fibroblast growth factor 18",
  "gene_symbol": "FGF18",
  "gene": "UniProtKB:O76093",
  "term_label": "growth factor activity"
}